detection of molecule of bacterial origin [GO:0032490] (biological process) Also known as: detection of bacteria associated molecule, detection of bacterial associated molecule, detection of bacterium associated molecule Relationships: is a type of response to molecule of bacterial origin [GO:0002237]; is a type of GO:0009593; is a type of detection of external biotic stimulus [GO:0098581] Definition: The series of events in which a stimulus from a molecule of bacterial origin is received and converted into a molecular signal. Subtypes: detection of lipopolysaccharide [GO:0032497], GO:0032499, GO:0042494, detection of lipoteichoic acid [GO:0070392] Sources: GOC:add, GOC:rl